floral meristem determinacy [GO:0010582] (biological process) Definition: The process in which a floral meristem becomes determinate (i.e. ceases to produce lateral organs and may or may not terminally differentiate). References: PMID:18441215 Relationships: is a type of GO:0003006; is a type of meristem determinacy [GO:0010022]; is part of GO:0009908